{
  "term_id": "GO:0008253",
  "gene_name": "5'-nucleotidase",
  "term_label": "5'-nucleotidase activity",
  "gene": "UniProtKB:P21589",
  "gene_symbol": "NT5E"
}